regulation of epithelial cell differentiation involved in kidney development [GO:2000696] (biological process) Relationships: is a type of regulation of epithelial cell differentiation [GO:0030856]; regulates GO:0035850 Sources: GOC:mtg_kidney_jan10, GOC:yaf Definition: Any process that modulates the frequency, rate or extent of epithelial cell differentiation involved in kidney development. Subtypes: regulation of mesenchymal to epithelial transition involved in metanephros morphogenesis [GO:0003339], regulation of nephron tubule epithelial cell differentiation [GO:0072182], GO:2000084, negative regulation of epithelial cell differentiation involved in kidney development [GO:2000697], positive regulation of epithelial cell differentiation involved in kidney development [GO:2000698]